{
  "gene_symbol": "COX6A2",
  "term_id": "GO:0045277",
  "term_label": "respiratory chain complex IV",
  "gene_name": "Cytochrome c oxidase subunit 6A2, mitochondrial",
  "gene": "UniProtKB:Q02221"
}